{
  "gene_symbol": "EIF1B",
  "term_id": "UNKNOWN:0002",
  "gene": "UniProtKB:O60739",
  "gene_name": "Eukaryotic translation initiation factor 1b",
  "term_label": "Unknown biological process"
}